{
  "gene_symbol": "TREML4",
  "gene": "UniProtKB:Q6UXN2",
  "term_label": "cell surface",
  "term_id": "GO:0009986",
  "gene_name": "Trem-like transcript 4 protein"
}